{
  "term_label": "DNA-binding transcription factor activity, RNA polymerase II-specific",
  "gene_symbol": "ZNF117",
  "gene_name": "Zinc finger protein 117",
  "term_id": "GO:0000981",
  "gene": "UniProtKB:Q03924"
}